{
  "term_label": "apical plasma membrane",
  "gene_symbol": "SLC4A7",
  "gene_name": "Sodium bicarbonate cotransporter 3",
  "gene": "UniProtKB:Q9Y6M7",
  "term_id": "GO:0016324"
}